{
  "gene": "UniProtKB:O00764",
  "gene_name": "Pyridoxal kinase",
  "term_id": "GO:0005829",
  "term_label": "cytosol",
  "gene_symbol": "PDXK"
}